acetyl-CoA C-acetyltransferase activity [GO:0003985] (molecular function) Sources: RHEA:21036 Also known as: acetoacetyl-CoA thiolase activity, acetyl coenzyme A thiolase activity Relationships: is a type of GO:0003988; is a type of C-acetyltransferase activity [GO:0016453] Definition: Catalysis of the reaction: 2 acetyl-CoA = CoA + acetoacetyl-CoA.